{
  "gene": "UniProtKB:P16152",
  "term_id": "UNKNOWN:0003",
  "term_label": "Unknown cellular component",
  "gene_name": "Carbonyl reductase [NADPH] 1",
  "gene_symbol": "CBR1"
}